{
  "term_id": "GO:0090385",
  "gene_name": "1-phosphatidylinositol 3-phosphate 5-kinase",
  "term_label": "phagosome-lysosome fusion",
  "gene_symbol": "PIKFYVE",
  "gene": "UniProtKB:Q9Y2I7"
}